{
  "term_label": "phosphatidylglycerol metabolic process",
  "gene_symbol": "PLA2G2C",
  "gene": "UniProtKB:Q5R387",
  "term_id": "GO:0046471",
  "gene_name": "Putative inactive group IIC secretory phospholipase A2"
}